{
  "gene_symbol": "OR4A15",
  "term_label": "plasma membrane",
  "gene_name": "Olfactory receptor 4A15",
  "term_id": "GO:0005886",
  "gene": "UniProtKB:Q8NGL6"
}